{
  "term_id": "GO:0072686",
  "gene_symbol": "KIFC1",
  "gene": "UniProtKB:Q9BW19",
  "gene_name": "Kinesin-like protein KIFC1",
  "term_label": "mitotic spindle"
}